N-cyclopropylammelide alkylamino hydrolase activity [GO:0034549] (molecular function) Relationships: is_a hydrolase activity, acting on carbon-nitrogen (but not peptide) bonds, in cyclic amidines [GO:0016814] Definition: Catalysis of the reaction: N-cyclopropylammelide + H2O = cyclopropylamine + cyanuric acid. Sources: UM-BBD_reactionID:r0827